{
  "term_label": "3',5'-cyclic-GMP phosphodiesterase activity",
  "term_id": "GO:0047555",
  "gene_symbol": "PDE4D",
  "gene_name": "cAMP-specific 3',5'-cyclic phosphodiesterase 4D",
  "gene": "UniProtKB:Q08499"
}